{
  "term_label": "acetylcholine-gated channel complex",
  "gene_name": "Acetylcholine receptor subunit gamma",
  "gene": "UniProtKB:P07510",
  "gene_symbol": "CHRNG",
  "term_id": "GO:0005892"
}